{
  "gene": "UniProtKB:Q8TDE3",
  "gene_symbol": "RNASE8",
  "gene_name": "Ribonuclease 8",
  "term_id": "GO:0050829",
  "term_label": "defense response to Gram-negative bacterium"
}